{
  "gene": "UniProtKB:P50570",
  "term_label": "microtubule",
  "gene_name": "Dynamin-2",
  "term_id": "GO:0005874",
  "gene_symbol": "DNM2"
}